{
  "gene_name": "Ubiquitin carboxyl-terminal hydrolase 35",
  "term_id": "GO:0005829",
  "term_label": "cytosol",
  "gene": "UniProtKB:Q9P2H5",
  "gene_symbol": "USP35"
}